{
  "gene_symbol": "GRAMD1A",
  "gene": "UniProtKB:Q96CP6",
  "term_label": "cholesterol transfer activity",
  "term_id": "GO:0120020",
  "gene_name": "Protein Aster-A"
}